{
  "term_label": "nucleus",
  "gene_symbol": "ZNF638",
  "gene_name": "Zinc finger protein 638",
  "gene": "UniProtKB:Q14966",
  "term_id": "GO:0005634"
}